{
  "term_id": "GO:0005615",
  "term_label": "extracellular space",
  "gene": "UniProtKB:P05230",
  "gene_name": "Fibroblast growth factor 1",
  "gene_symbol": "FGF1"
}